protease localization to T cell secretory granule [GO:0033375] (biological process) Definition: Any process in which a protease is transported to, or maintained in, a location within a secretory granule in a T cell. Also known as: protease localisation in T cell secretory granule, protease localization in T cell secretory granule, protease localization in T lymphocyte secretory granule, protease localization in T-cell secretory granule, protease localization in T-lymphocyte secretory granule Sources: GOC:mah Relationships: is a type of protein localization to T cell secretory granule [GO:0033374] Subtypes: granzyme B localization to T cell secretory granule [GO:0033380]